{
  "gene": "UniProtKB:Q9H497",
  "term_id": "GO:0005635",
  "term_label": "nuclear envelope",
  "gene_symbol": "TOR3A",
  "gene_name": "Torsin-3A"
}